renal system process [GO:0003014] (biological process) Regulation: regulated by regulation of renal system process [GO:0098801] Subtypes: GO:0003071, renal water homeostasis [GO:0003091], renal sodium ion transport [GO:0003096], GO:0003097, GO:0035809, micturition [GO:0060073], renal absorption [GO:0070293], renal filtration [GO:0097205], renal tubular secretion [GO:0097254] Relationships: is a type of GO:0003008 Definition: An organ system process carried out by any of the organs or tissues of the renal system. The renal system maintains fluid balance, and contributes to electrolyte balance, acid/base balance, and disposal of nitrogenous waste products. In humans, the renal system comprises a pair of kidneys, a pair of ureters, urinary bladder, urethra, sphincter muscle and associated blood vessels; in other species, the renal system may comprise related structures (e.g., nephrocytes and malpighian tubules in Drosophila). Also known as: excretory system process, kidney system process Sources: GOC:cjm, GOC:mtg_cardio, GOC:mtg_kidney_jan10